nephron tubule morphogenesis [GO:0072078] (biological process) Subtypes: pronephric nephron tubule morphogenesis [GO:0039008], GO:0072156, proximal tubule morphogenesis [GO:0072158], mesonephric tubule morphogenesis [GO:0072171], metanephric nephron tubule morphogenesis [GO:0072282] Sources: GOC:mtg_kidney_jan10 Definition: The process in which the anatomical structures of a nephron tubule are generated and organized. A nephron tubule is an epithelial tube that is part of the nephron, the functional part of the kidney. Relationships: is a type of GO:0061333; is a type of nephron epithelium morphogenesis [GO:0072088]; is part of nephron tubule development [GO:0072080]